negative regulation of convergent extension involved in notochord morphogenesis [GO:1904137] (biological process) Definition: Any process that stops, prevents or reduces the frequency, rate or extent of convergent extension involved in notochord morphogenesis. References: PMID:24892953 Sources: GOC:TermGenie, GOC:dph, GO_REF:0000058 Also known as: down regulation of convergent extension involved in notochord morphogenesis, down-regulation of convergent extension involved in notochord morphogenesis, downregulation of convergent extension involved in notochord morphogenesis, inhibition of convergent extension involved in notochord morphogenesis Relationships: is a type of negative regulation of convergent extension involved in gastrulation [GO:1904104]; is a type of regulation of convergent extension involved in notochord morphogenesis [GO:1904136]; negatively regulates GO:1904126